choline trimethylamine lyase activity [GO:0120525] (molecular function) Note: Note that this term has a MetaCyc pathway reference as the pathway only has a single step. Relationships: is a type of carbon-nitrogen lyase activity [GO:0016840] Sources: RHEA:35095 Definition: Catalysis of the reaction: choline = acetaldehyde + trimethylamine.